positive regulation of motile cilium assembly [GO:1905505] (biological process) Relationships: is a type of GO:0045724; is a type of regulation of motile cilium assembly [GO:1905503]; positively regulates motile cilium assembly [GO:0044458] Also known as: activation of motile primary cilia assembly, activation of motile primary cilia formation, activation of motile primary cilium assembly, activation of motile primary cilium formation, activation of nodal cilium assembly, activation of nodal cilium formation, positive regulation of motile primary cilia assembly, positive regulation of motile primary cilia formation, positive regulation of motile primary cilium assembly, positive regulation of motile primary cilium formation, positive regulation of nodal cilium assembly, positive regulation of nodal cilium formation, up regulation of motile primary cilia assembly, up regulation of motile primary cilia formation, up regulation of motile primary cilium assembly, up regulation of motile primary cilium formation, up regulation of nodal cilium assembly, up regulation of nodal cilium formation, up-regulation of motile primary cilia assembly, up-regulation of motile primary cilia formation, up-regulation of motile primary cilium assembly, up-regulation of motile primary cilium formation, up-regulation of nodal cilium assembly, up-regulation of nodal cilium formation, upregulation of motile primary cilia assembly, upregulation of motile primary cilia formation, upregulation of motile primary cilium assembly, upregulation of motile primary cilium formation, upregulation of nodal cilium assembly, upregulation of nodal cilium formation References: PMID:25294941 Sources: GOC:TermGenie, GOC:cilia, GOC:krc, GO_REF:0000058 Definition: Any process that activates or increases the frequency, rate or extent of motile cilium assembly.